{
  "term_id": "GO:0042742",
  "gene": "UniProtKB:P0DP73",
  "gene_name": "Beta-defensin 130B",
  "gene_symbol": "DEFB130B",
  "term_label": "defense response to bacterium"
}